{
  "gene": "UniProtKB:Q9H254",
  "term_id": "GO:0042995",
  "term_label": "cell projection",
  "gene_name": "Spectrin beta chain, non-erythrocytic 4",
  "gene_symbol": "SPTBN4"
}